monolayer-surrounded lipid storage body outer lipid monolayer [GO:0034430] (cellular component) Definition: The single layer of phopholipids surrounding a lipid storage body. Relationships: is a type of organelle-enclosing lipid monolayer [GO:0034646]; is part of cytoplasm [GO:0005737]; is part of monolayer-surrounded lipid storage body [GO:0012511] Also known as: lipid storage body surface lipid monolayer, oil body outer lipid monolayer, oleosome outer lipid monolayer, spherosome outer lipid monolayer, lipid droplet outer lipid monolayer Sources: GOC:rph